{
  "term_id": "UNKNOWN:0003",
  "gene_symbol": "TMSB15C",
  "term_label": "Unknown cellular component",
  "gene_name": "Thymosin beta-15C",
  "gene": "UniProtKB:P0DX04"
}